{
  "gene_symbol": "CARD14",
  "gene_name": "Caspase recruitment domain-containing protein 14",
  "gene": "UniProtKB:Q9BXL6",
  "term_label": "regulation of immune response",
  "term_id": "GO:0050776"
}